response to acrylamide [GO:1903937] (biological process) Relationships: is a type of response to nitrogen compound [GO:1901698]; is a type of response to oxygen-containing compound [GO:1901700] References: PMID:16292499 Sources: GOC:TermGenie, GO_REF:0000071 Subtypes: GO:1903938 Definition: Any process that results in a change in state or activity of a cell or an organism (in terms of movement, secretion, enzyme production, gene expression, etc.) as a result of an acrylamide stimulus.